{
  "gene_symbol": "NRIP1",
  "gene": "UniProtKB:P48552",
  "term_id": "GO:0035259",
  "gene_name": "Nuclear receptor-interacting protein 1",
  "term_label": "nuclear glucocorticoid receptor binding"
}